histone H3K18 decrotonylase activity [GO:0170012] (MF) References: PMID:34927582 Note: Comment: Note that the residue position corresponds to the canonical human H3 histone (UniProtKB:P84243); this residue is conserved across all eukaryotes. Residue 1 is the first residue following removal of the initiating Methionine (Met). Note that each histone is encoded by multiple genes, and sequences may vary across different genes within an organism. Definition: Catalysis of the reaction: H2O + N6-(2E)-butenoyl-L-lysyl-[histone H3 position 18] + NAD+ = 2''-O-(2E)-but-2-enoyl-ADP-D-ribose + L-lysyl-[histone H3] + nicotinamide. Relationships: is a type of histone decrotonylase activity, NAD-dependent [GO:0160012]